{
  "gene_symbol": "ARMS2",
  "term_label": "Unknown cellular component",
  "term_id": "UNKNOWN:0003",
  "gene": "UniProtKB:P0C7Q2",
  "gene_name": "Age-related maculopathy susceptibility protein 2"
}